negative regulation of L-leucine import across plasma membrane [GO:1905533] (biological process) Definition: Any process that stops, prevents or reduces the frequency, rate or extent of L-leucine import across plasma membrane. Also known as: down regulation of L-leucine import into cell, down-regulation of L-leucine import into cell, downregulation of L-leucine import into cell, negative regulation of L-leucine import into cell, inhibition of leucine import into cell References: PMID:10467003 Sources: GOC:TermGenie, GO_REF:0000058 Subtypes: negative regulation of leucine import in response to ammonium ion [GO:0060360] Relationships: is_a negative regulation of organic acid transport [GO:0032891]; is a type of negative regulation of transmembrane transport [GO:0034763]; is a type of negative regulation of amino acid transport [GO:0051956]; is a type of regulation of L-leucine import across plasma membrane [GO:1905532]; negatively regulates GO:1903801